regulation of antimicrobial peptide secretion [GO:0002794] (biological process) Relationships: is a type of regulation of antimicrobial peptide production [GO:0002784]; is_a regulation of peptide secretion [GO:0002791]; regulates GO:0002776 Subtypes: GO:0002795, positive regulation of antimicrobial peptide secretion [GO:0002796], regulation of antibacterial peptide secretion [GO:0002797], regulation of antifungal peptide secretion [GO:0002800] Sources: GOC:add Definition: Any process that modulates the frequency, rate, or extent of antimicrobial peptide secretion.